{
  "gene_name": "Myeloid-associated differentiation marker-like protein 2",
  "term_id": "UNKNOWN:0002",
  "gene_symbol": "MYADML2",
  "term_label": "Unknown biological process",
  "gene": "UniProtKB:A6NDP7"
}